interleukin-2 receptor binding [GO:0005134] (molecular function) Sources: GOC:ai Definition: Binding to an interleukin-2 receptor. Also known as: IL-2, interleukin-2 receptor ligand Relationships: is a type of cytokine receptor binding [GO:0005126]; is a type of growth factor receptor binding [GO:0070851]